{
  "gene_symbol": "SLC39A10",
  "gene_name": "Zinc transporter ZIP10",
  "term_label": "zinc ion import across plasma membrane",
  "gene": "UniProtKB:Q9ULF5",
  "term_id": "GO:0071578"
}